positive regulation of adult salivary gland boundary specification [GO:0045711] (biological process) Sources: GOC:go_curators, GOC:tb Also known as: positive regulation of adult salivary gland determination, up regulation of adult salivary gland determination, up-regulation of adult salivary gland determination, upregulation of adult salivary gland determination, activation of adult salivary gland determination, stimulation of adult salivary gland determination Relationships: is a type of GO:0045706; is a type of regulation of adult salivary gland boundary specification [GO:0045707]; positively regulates adult salivary gland boundary specification [GO:0007434] Definition: Any process that activates or increases the frequency, rate or extent of salivary gland determination in an adult organism.